{
  "term_id": "GO:0001228",
  "gene": "UniProtKB:O00570",
  "term_label": "DNA-binding transcription activator activity, RNA polymerase II-specific",
  "gene_name": "Transcription factor SOX-1",
  "gene_symbol": "SOX1"
}